UDP-L-arabinose biosynthetic process [GO:0033358] (biological process) Sources: GOC:mah, MetaCyc:PWY-82 Relationships: is a type of GO:0009226; is_a UDP-L-arabinose metabolic process [GO:0033356] Also known as: UDP-L-arabinose anabolism, UDP-L-arabinose biosynthesis, UDP-L-arabinose formation, UDP-L-arabinose synthesis Definition: The chemical reactions and pathways resulting in the formation of UDP-L-arabinose, uridinediphosphoarabinose, a substance composed of arabinose in glycosidic linkage with uridine diphosphate.